{
  "gene_symbol": "ITPR2",
  "gene_name": "Inositol 1,4,5-trisphosphate receptor type 2",
  "term_label": "secretory granule membrane",
  "gene": "UniProtKB:Q14571",
  "term_id": "GO:0030667"
}